{
  "term_id": "GO:0005634",
  "term_label": "nucleus",
  "gene_symbol": "CEBPZ",
  "gene": "UniProtKB:Q03701",
  "gene_name": "CCAAT_enhancer-binding protein zeta"
}